{
  "gene_name": "Double homeobox protein 4C",
  "gene_symbol": "DUX4L9",
  "gene": "UniProtKB:Q6RFH8",
  "term_id": "GO:0000977",
  "term_label": "RNA polymerase II transcription regulatory region sequence-specific DNA binding"
}